{
  "gene_name": "ATP-binding cassette sub-family B member 6",
  "term_id": "GO:0015439",
  "gene": "UniProtKB:Q9NP58",
  "term_label": "ABC-type heme transporter activity",
  "gene_symbol": "ABCB6"
}